{
  "gene_symbol": "IGKJ5",
  "term_id": "UNKNOWN:0001",
  "gene_name": "Immunoglobulin kappa joining 5 (Fragment)",
  "term_label": "Unknown molecular function",
  "gene": "UniProtKB:A0A0A0MTA3"
}